cysteine-conjugate transaminase activity [GO:0047802] (molecular function) Definition: Catalysis of the reaction: 2-oxoglutarate + S-(4-bromophenyl)-L-cysteine = (4-bromophenylsulfanyl)pyruvate + L-glutamate. Sources: EC:2.6.1.75, RHEA:13485 Relationships: is a type of transaminase activity [GO:0008483] Also known as: S-(4-bromophenyl)-L-cysteine:2-oxoglutarate aminotransferase activity, cysteine conjugate aminotransferase activity, cysteine-conjugate alpha-ketoglutarate transaminase (CAT-1)